phosphatidyltransferase activity [GO:0030572] (molecular function) Definition: Catalysis of the reaction involving the transfer of a phosphatidate (otherwise known as diacylglycerol 3-phosphosphate) group. Sources: GOC:mb Subtypes: cardiolipin synthase activity [GO:0008808], cardiolipin synthase (CMP-forming) [GO:0043337], GO:0090483 Relationships: is a type of phosphotransferase activity, for other substituted phosphate groups [GO:0016780]